{
  "gene_name": "Bystin",
  "term_label": "snoRNA binding",
  "term_id": "GO:0030515",
  "gene_symbol": "BYSL",
  "gene": "UniProtKB:Q13895"
}